{
  "gene_name": "E3 ubiquitin-protein ligase RNF180",
  "term_id": "GO:0042428",
  "term_label": "serotonin metabolic process",
  "gene_symbol": "RNF180",
  "gene": "UniProtKB:Q86T96"
}